arabinogalactan binding [GO:2001085] (molecular function) Relationships: is a type of polysaccharide binding [GO:0030247] Sources: GOC:mengo_curators Definition: Binding to arabinogalactan.